{
  "gene_symbol": "JUN",
  "term_id": "GO:0042127",
  "term_label": "regulation of cell population proliferation",
  "gene_name": "Transcription factor Jun",
  "gene": "UniProtKB:P05412"
}